{
  "gene_symbol": "FOXO3B",
  "term_id": "GO:0005634",
  "gene": "UniProtKB:A0A2Z4LIS9",
  "gene_name": "Forkhead box protein O3B",
  "term_label": "nucleus"
}